regulation of mineralocorticoid secretion [GO:2000855] (biological process) Sources: GOC:sl Definition: Any process that modulates the frequency, rate or extent of mineralocorticoid secretion. Subtypes: negative regulation of mineralocorticoid secretion [GO:2000856], positive regulation of mineralocorticoid secretion [GO:2000857], regulation of aldosterone secretion [GO:2000858] Relationships: is a type of regulation of corticosteroid hormone secretion [GO:2000846]; regulates mineralocorticoid secretion [GO:0035931]